{
  "gene_name": "Neuroepithelial cell-transforming gene 1 protein",
  "term_id": "GO:0035025",
  "gene_symbol": "NET1",
  "term_label": "positive regulation of Rho protein signal transduction",
  "gene": "UniProtKB:Q7Z628"
}